{
  "term_id": "GO:0036488",
  "term_label": "CHOP-C/EBP complex",
  "gene_name": "DNA damage-inducible transcript 3 protein",
  "gene_symbol": "DDIT3",
  "gene": "UniProtKB:P35638"
}